{
  "gene": "UniProtKB:Q5M9N0",
  "term_label": "Unknown biological process",
  "term_id": "UNKNOWN:0002",
  "gene_symbol": "CCDC158",
  "gene_name": "Coiled-coil domain-containing protein 158"
}